synaptobrevin 2-SNAP-25-syntaxin-3 complex [GO:0070046] (cellular component) Relationships: is a type of SNARE complex [GO:0031201] Definition: A SNARE complex that contains synaptobrevin 2 (VAMP2), SNAP-25, and syntaxin 3 (or orthologs thereof). Also known as: SNARE complex (Stx3, Snap25, Vamp2), Stx3-Snap25-Vamp2 complex References: PMID:10336434